rRNA (adenine-N6,N6-)-dimethyltransferase activity [GO:0000179] (molecular function) Relationships: is_a N-methyltransferase activity [GO:0008170]; is a type of GO:0016433 Also known as: 18S rRNA dimethylase activity, S-adenosylmethionine-6-N', N'-adenosyl(rRNA) dimethyltransferase activity, dimethyladenosine transferase activity References: PMID:10690410 Sources: ISBN:1555811337 Definition: Catalysis of the dimethylation of two adjacent adenine residues in a rRNA, using S-adenosyl-L-methionine as a methyl donor. Subtypes: 16S rRNA (adenine(1518)-N(6)/adenine(1519)-N(6))-dimethyltransferase activity [GO:0052908], 18S rRNA (adenine(1779)-N(6)/adenine(1780)-N(6))-dimethyltransferase activity [GO:0052909]